{
  "term_label": "G protein-coupled receptor activity",
  "gene_symbol": "ADGRD2",
  "gene_name": "Adhesion G-protein coupled receptor D2",
  "term_id": "GO:0004930",
  "gene": "UniProtKB:Q7Z7M1"
}